positive regulation of inhibitory postsynaptic potential [GO:0097151] (biological process) References: PMID:18550748 Sources: GOC:BHF, GOC:sjp Also known as: positive regulation of IPSP, positive regulation of inhibitory post-synaptic membrane potential Relationships: is a type of GO:0031646; is a type of modulation of inhibitory postsynaptic potential [GO:0098828]; positively regulates inhibitory postsynaptic potential [GO:0060080] Definition: Any process that activates or increases the frequency, rate or extent of inhibitory postsynaptic potential (IPSP). IPSP is a temporary decrease in postsynaptic membrane potential due to the flow of negatively charged ions into the postsynaptic cell. The flow of ions that causes an IPSP is an inhibitory postsynaptic current (IPSC) and makes it more difficult for the neuron to fire an action potential.